{
  "term_label": "potassium channel regulator activity",
  "gene_symbol": "KCNS1",
  "term_id": "GO:0015459",
  "gene_name": "Potassium voltage-gated channel subfamily S member 1",
  "gene": "UniProtKB:Q96KK3"
}